negative regulation of inner ear auditory receptor cell differentiation [GO:0045608] (biological process) Definition: Any process that stops, prevents, or reduces the frequency, rate or extent of auditory hair cell differentiation. Sources: GOC:go_curators Also known as: down regulation of auditory receptor cell differentiation, down-regulation of auditory receptor cell differentiation, downregulation of auditory receptor cell differentiation, negative regulation of auditory hair cell differentiation, inhibition of auditory receptor cell differentiation, negative regulation of auditory receptor cell differentiation Relationships: is a type of negative regulation of epidermal cell differentiation [GO:0045605]; is a type of regulation of inner ear auditory receptor cell differentiation [GO:0045607]; is a type of GO:2000981; negatively regulates inner ear auditory receptor cell differentiation [GO:0042491] Subtypes: GO:0009999